{
  "term_label": "membrane",
  "term_id": "GO:0016020",
  "gene_symbol": "KCNA5",
  "gene_name": "Potassium voltage-gated channel subfamily A member 5",
  "gene": "UniProtKB:P22460"
}